chondro-4-sulfatase activity [GO:0033887] (molecular function) Definition: Catalysis of the reaction: 4-deoxy-beta-D-gluc-4-enuronosyl-(1->3)-N-acetyl-D-galactosamine 4-sulfate + H2O = 4-deoxy-beta-D-gluc-4-enuronosyl-(1->3)-N-acetyl-D-galactosamine + H+ + sulfate. Sources: EC:3.1.6.9, RHEA:11444 Relationships: is a type of GO:0008484 Also known as: 4-deoxy-beta-D-gluc-4-enuronosyl-(1,3)-N-acetyl-D-galactosamine-4-sulfate 4-sulfohydrolase activity